{
  "term_label": "external side of plasma membrane",
  "gene_name": "Cytokine receptor-like factor 1",
  "gene_symbol": "CRLF1",
  "term_id": "GO:0009897",
  "gene": "UniProtKB:O75462"
}